{
  "gene_symbol": "NEUROG2",
  "term_label": "E-box binding",
  "gene": "UniProtKB:Q9H2A3",
  "term_id": "GO:0070888",
  "gene_name": "Neurogenin-2"
}